{
  "gene": "UniProtKB:Q8IWE5",
  "term_id": "GO:0019894",
  "gene_symbol": "PLEKHM2",
  "gene_name": "Pleckstrin homology domain-containing family M member 2",
  "term_label": "kinesin binding"
}